{
  "gene_symbol": "VPS11",
  "gene": "UniProtKB:Q9H270",
  "gene_name": "Vacuolar protein sorting-associated protein 11 homolog",
  "term_label": "HOPS complex",
  "term_id": "GO:0030897"
}